{
  "term_label": "mitochondrion",
  "gene": "UniProtKB:Q9ULR3",
  "term_id": "GO:0005739",
  "gene_symbol": "PPM1H",
  "gene_name": "Protein phosphatase 1H"
}